{
  "gene": "UniProtKB:Q96DT0",
  "gene_name": "Galectin-12",
  "term_id": "GO:0097193",
  "gene_symbol": "LGALS12",
  "term_label": "intrinsic apoptotic signaling pathway"
}